{
  "gene_symbol": "CSGALNACT1",
  "term_label": "glucuronosyl-N-acetylgalactosaminyl-proteoglycan 4-beta-N-acetylgalactosaminyltransferase activity",
  "gene_name": "Chondroitin sulfate N-acetylgalactosaminyltransferase 1",
  "term_id": "GO:0047238",
  "gene": "UniProtKB:Q8TDX6"
}